{
  "term_label": "positive regulation of brown fat cell differentiation",
  "gene_name": "Meteorin-like protein",
  "gene_symbol": "METRNL",
  "gene": "UniProtKB:Q641Q3",
  "term_id": "GO:0090336"
}